{
  "gene_symbol": "SYT2",
  "term_id": "GO:0017158",
  "gene_name": "Synaptotagmin-2",
  "term_label": "regulation of calcium ion-dependent exocytosis",
  "gene": "UniProtKB:Q8N9I0"
}